{
  "gene_name": "Protein FAM117B",
  "gene_symbol": "FAM117B",
  "term_label": "Unknown cellular component",
  "term_id": "UNKNOWN:0003",
  "gene": "UniProtKB:Q6P1L5"
}